{
  "gene_name": "Putative melanoma-associated antigen 5P",
  "term_label": "Unknown cellular component",
  "gene": "UniProtKB:P43359",
  "term_id": "UNKNOWN:0003",
  "gene_symbol": "MAGEA5P"
}